purine ribonucleotide biosynthetic process [GO:0009152] (biological process) Definition: The chemical reactions and pathways resulting in the formation of a purine ribonucleotide, a compound consisting of ribonucleoside (a purine base linked to a ribose sugar) esterified with a phosphate group at either the 3' or 5'-hydroxyl group of the sugar. Also known as: purine ribonucleotide anabolism, purine ribonucleotide biosynthesis, purine ribonucleotide formation, purine ribonucleotide synthesis Subtypes: AMP biosynthetic process [GO:0006167], cAMP biosynthetic process [GO:0006171], ADP biosynthetic process [GO:0006172], GO:0006177, GO:0006182, GTP biosynthetic process [GO:0006183], IMP biosynthetic process [GO:0006188], ATP biosynthetic process [GO:0006754], GO:0015970, guanosine pentaphosphate biosynthetic process [GO:0015973], GO:0019361, ITP biosynthetic process [GO:0046042], GO:0046708, GDP biosynthetic process [GO:0046711], 3'-phosphoadenosine 5'-phosphosulfate biosynthetic process [GO:0050428], GO:0097293, purine ribonucleotide salvage [GO:0106380] Sources: GOC:go_curators, ISBN:0198506732 Relationships: is a type of purine nucleotide biosynthetic process [GO:0006164]; is a type of purine ribonucleotide metabolic process [GO:0009150]; is a type of ribonucleotide biosynthetic process [GO:0009260]